{
  "gene_name": "MAGE-like protein 2",
  "gene": "UniProtKB:Q9UJ55",
  "term_id": "UNKNOWN:0001",
  "term_label": "Unknown molecular function",
  "gene_symbol": "MAGEL2"
}